{
  "term_id": "GO:0006357",
  "gene": "UniProtKB:P31269",
  "term_label": "regulation of transcription by RNA polymerase II",
  "gene_name": "Homeobox protein Hox-A9",
  "gene_symbol": "HOXA9"
}